{
  "term_label": "regulation of transcription by RNA polymerase II",
  "term_id": "GO:0006357",
  "gene_name": "Cyclic AMP-responsive element-binding protein 3-like protein 1",
  "gene": "UniProtKB:Q96BA8",
  "gene_symbol": "CREB3L1"
}